{
  "gene": "UniProtKB:Q8NBU5",
  "term_label": "Unknown molecular function",
  "term_id": "UNKNOWN:0001",
  "gene_symbol": "ATAD1",
  "gene_name": "Outer mitochondrial transmembrane helix translocase"
}